{
  "gene_symbol": "EXOSC8",
  "term_label": "rRNA catabolic process",
  "gene": "UniProtKB:Q96B26",
  "term_id": "GO:0016075",
  "gene_name": "Exosome complex component RRP43"
}